{
  "term_id": "GO:0000400",
  "gene_name": "DNA repair protein RAD51 homolog 3",
  "gene": "UniProtKB:O43502",
  "gene_symbol": "RAD51C",
  "term_label": "four-way junction DNA binding"
}